{
  "gene": "UniProtKB:Q8NBL1",
  "gene_symbol": "POGLUT1",
  "term_label": "UDP-xylosyltransferase activity",
  "gene_name": "Protein O-glucosyltransferase 1",
  "term_id": "GO:0035252"
}